{
  "gene_name": "Transcription factor SOX-8",
  "gene": "UniProtKB:P57073",
  "term_label": "peripheral nervous system development",
  "term_id": "GO:0007422",
  "gene_symbol": "SOX8"
}